cellular response to hepatocyte growth factor stimulus [GO:0035729] (biological process) Definition: Any process that results in a change in state or activity of a cell (in terms of movement, secretion, enzyme production, gene expression, etc.) as a result of a hepatocyte growth factor stimulus. Sources: GOC:bf Also known as: cellular response to HGF stimulus Relationships: is a type of response to hepatocyte growth factor [GO:0035728]; is a type of GO:0071363 Regulation: regulated by GO:2001112; negatively regulated by GO:2001113; positively regulated by positive regulation of cellular response to hepatocyte growth factor stimulus [GO:2001114]